{
  "gene_name": "Calcium channel flower homolog",
  "term_label": "Unknown molecular function",
  "gene_symbol": "CACFD1",
  "term_id": "UNKNOWN:0001",
  "gene": "UniProtKB:Q9UGQ2"
}